positive regulation of granulocyte macrophage colony-stimulating factor production [GO:0032725] (biological process) Definition: Any process that activates or increases the frequency, rate, or extent of granulocyte macrophage colony-stimulating factor production. Also known as: positive regulation of GM-CSF production, positive regulation of granulocyte macrophage colony stimulating factor production, up regulation of granulocyte macrophage colony-stimulating factor production, up-regulation of granulocyte macrophage colony-stimulating factor production, upregulation of granulocyte macrophage colony-stimulating factor production, activation of granulocyte macrophage colony-stimulating factor production, positive regulation of granulocyte macrophage colony-stimulating factor biosynthetic process, stimulation of granulocyte macrophage colony-stimulating factor production Sources: GOC:mah Relationships: is a type of positive regulation of cytokine production [GO:0001819]; is a type of regulation of granulocyte macrophage colony-stimulating factor production [GO:0032645]; is a type of positive regulation of protein metabolic process [GO:0051247]; positively regulates granulocyte macrophage colony-stimulating factor production [GO:0032604]